{
  "gene_name": "BAG family molecular chaperone regulator 5",
  "gene_symbol": "BAG5",
  "term_label": "protein-folding chaperone binding",
  "term_id": "GO:0051087",
  "gene": "UniProtKB:Q9UL15"
}